response to follicle-stimulating hormone [GO:0032354] (biological process) Also known as: response to FSH stimulus, response to follicle stimulating hormone stimulus, response to follicle-stimulating hormone stimulus Definition: Any process that results in a change in state or activity of a cell or an organism (in terms of movement, secretion, enzyme production, gene expression, etc.) as a result of a follicle-stimulating hormone stimulus. Relationships: is a type of GO:0034698 Subtypes: cellular response to follicle-stimulating hormone stimulus [GO:0071372] Sources: GOC:mah